rRNA 2'-O-ribose methylation guide activity [GO:0030562] (molecular function) Relationships: is a type of rRNA modification guide activity [GO:0030556]; is a type of GO:0030561 References: PMID:12457565 Sources: GOC:mah Definition: Specifies the site of 2'-O-ribose methylation in an rRNA molecule by base pairing with a short sequence around the target residue. Note: Note that this term describes the activity of a nucleic acid, usually RNA, gene product that interacts with other RNA molecules via base pairing; it should not be used to annotate proteins.